{
  "gene_symbol": "TTC1",
  "term_id": "UNKNOWN:0003",
  "gene_name": "Tetratricopeptide repeat protein 1",
  "gene": "UniProtKB:Q99614",
  "term_label": "Unknown cellular component"
}